cellular response to genistein [GO:0071412] (biological process) Definition: Any process that results in a change in state or activity of a cell (in terms of movement, secretion, enzyme production, gene expression, etc.) as a result of a genistein stimulus. Sources: GOC:mah Relationships: is a type of response to genistein [GO:0033595]; is_a cellular response to hydroxyisoflavone [GO:0071413]